cellulosome [GO:0043263] (cellular component) Also known as: scaffoldin complex Relationships: is a type of extracellular membraneless organelle [GO:0043264] Definition: An extracellular multi-enzyme complex containing up to 11 different enzymes aligned on a non-catalytic scaffolding glycoprotein. Functions to hydrolyze cellulose. References: PMID:11601609, PMID:15197390, PMID:20373916 Sources: GOC:jl